D(-)-tartrate dehydratase activity [GO:0047808] (molecular function) Relationships: is a type of hydro-lyase activity [GO:0016836] Also known as: (S,S)-tartrate hydro-lyase (oxaloacetate-forming), (S,S)-tartrate hydro-lyase activity, D-tartrate dehydratase activity Sources: EC:4.2.1.81, RHEA:18289 Definition: Catalysis of the reaction: D-tartrate = H2O + oxaloacetate.